{
  "gene_name": "Progesterone receptor",
  "term_id": "GO:0000785",
  "gene": "UniProtKB:P06401",
  "gene_symbol": "PGR",
  "term_label": "chromatin"
}